{
  "gene_symbol": "ZNF542P",
  "term_label": "Unknown cellular component",
  "gene_name": "Putative zinc finger protein 542",
  "gene": "UniProtKB:Q5EBM4",
  "term_id": "UNKNOWN:0003"
}